{
  "gene": "UniProtKB:O95810",
  "term_id": "GO:0005737",
  "term_label": "cytoplasm",
  "gene_symbol": "CAVIN2",
  "gene_name": "Caveolae-associated protein 2"
}